regulation of muscle filament sliding [GO:0032971] (biological process) Definition: Any process that modulates the frequency, rate or extent of muscle filament sliding. Subtypes: regulation of muscle filament sliding involved in regulation of the velocity of shortening in skeletal muscle contraction [GO:0014880], regulation of muscle filament sliding speed [GO:0032972], negative regulation of muscle filament sliding [GO:1904113], GO:1904114 Relationships: is a type of regulation of muscle contraction [GO:0006937]; is a type of regulation of intracellular transport [GO:0032386]; is a type of GO:1903115; regulates muscle filament sliding [GO:0030049] Sources: GOC:ecd